{
  "term_label": "detection of chemical stimulus involved in sensory perception of smell",
  "gene_name": "Olfactory receptor 2F2",
  "gene": "UniProtKB:O95006",
  "gene_symbol": "OR2F2",
  "term_id": "GO:0050911"
}